{
  "term_label": "growth factor activity",
  "gene_name": "Artemin",
  "gene": "UniProtKB:Q5T4W7",
  "gene_symbol": "ARTN",
  "term_id": "GO:0008083"
}